{
  "term_id": "GO:0000479",
  "gene_name": "Ribosome biogenesis protein BMS1 homolog",
  "gene": "UniProtKB:Q14692",
  "gene_symbol": "BMS1",
  "term_label": "endonucleolytic cleavage of tricistronic rRNA transcript (SSU-rRNA, 5.8S rRNA, LSU-rRNA)"
}